{
  "term_id": "GO:0034727",
  "gene": "UniProtKB:Q9Y4P1",
  "term_label": "piecemeal microautophagy of the nucleus",
  "gene_symbol": "ATG4B",
  "gene_name": "Cysteine protease ATG4B"
}